{
  "gene": "UniProtKB:Q8TF44",
  "term_label": "Unknown molecular function",
  "gene_symbol": "C2CD4C",
  "term_id": "UNKNOWN:0001",
  "gene_name": "C2 calcium-dependent domain-containing protein 4C"
}